histone H3 kinase activity [GO:0140996] (molecular function) Relationships: is a type of histone kinase activity [GO:0035173] Subtypes: GO:0035175, histone H3Y41 kinase activity [GO:0035401], histone H3T11 kinase activity [GO:0035402], histone H3T6 kinase activity [GO:0035403], histone H3S28 kinase activity [GO:0044022], histone H3T3 kinase activity [GO:0072354], histone H3S57 kinase activity [GO:0140855], GO:0140857 References: PMID:25303536 Definition: Catalysis of the transfer of a phosphate group to a histone H3.